{
  "term_label": "intracellular calcium ion homeostasis",
  "gene": "UniProtKB:Q969S6",
  "gene_symbol": "TMEM203",
  "gene_name": "Transmembrane protein 203",
  "term_id": "GO:0006874"
}